negative regulation of CD8-positive, alpha-beta cytotoxic T cell extravasation [GO:2000453] (biological process) Definition: Any process that stops, prevents or reduces the frequency, rate or extent of CD8-positive, alpha-beta cytotoxic T cell extravasation. Relationships: is a type of negative regulation of CD8-positive, alpha-beta T cell extravasation [GO:2000450]; is a type of regulation of CD8-positive, alpha-beta cytotoxic T cell extravasation [GO:2000452]; negatively regulates CD8-positive, alpha-beta cytotoxic T cell extravasation [GO:0035698] Sources: GOC:obol